{
  "gene_symbol": "SERINC2",
  "gene": "UniProtKB:Q96SA4",
  "gene_name": "Serine incorporator 2",
  "term_label": "membrane",
  "term_id": "GO:0016020"
}